{
  "gene_name": "Plakophilin-1",
  "gene": "UniProtKB:Q13835",
  "gene_symbol": "PKP1",
  "term_label": "cytoplasm",
  "term_id": "GO:0005737"
}